{
  "term_label": "zinc ion binding",
  "term_id": "GO:0008270",
  "gene_symbol": "SEC24A",
  "gene": "UniProtKB:O95486",
  "gene_name": "Protein transport protein Sec24A"
}